{
  "gene_name": "Putative uncharacterized protein C19orf81",
  "term_id": "UNKNOWN:0001",
  "gene_symbol": "C19orf81",
  "term_label": "Unknown molecular function",
  "gene": "UniProtKB:C9J6K1"
}